{
  "gene_name": "Defensin-6",
  "gene_symbol": "DEFA6",
  "term_label": "disruption of plasma membrane integrity in another organism",
  "term_id": "GO:0051673",
  "gene": "UniProtKB:Q01524"
}